capsular-polysaccharide endo-1,3-alpha-galactosidase activity [GO:0033921] (molecular function) Sources: EC:3.2.1.87 Relationships: is a type of galactosidase activity [GO:0015925] Also known as: aerobacter-capsular-polysaccharide galactohydrolase activity, capsular polysaccharide galactohydrolase activity, polysaccharide depolymerase activity Definition: Catalysis of the random hydrolysis of (1->3)-alpha-D-galactosidic linkages in Aerobacter aerogenes capsular polysaccharide.